{
  "gene": "UniProtKB:Q14114",
  "term_label": "Unknown molecular function",
  "term_id": "UNKNOWN:0001",
  "gene_name": "Low-density lipoprotein receptor-related protein 8",
  "gene_symbol": "LRP8"
}